{
  "term_id": "GO:0007059",
  "term_label": "chromosome segregation",
  "gene": "UniProtKB:Q69YH5",
  "gene_name": "Cell division cycle-associated protein 2",
  "gene_symbol": "CDCA2"
}